{
  "gene_symbol": "PAN2",
  "term_label": "nuclear-transcribed mRNA poly(A) tail shortening",
  "gene_name": "PAN2-PAN3 deadenylation complex catalytic subunit PAN2",
  "term_id": "GO:0000289",
  "gene": "UniProtKB:Q504Q3"
}